{
  "gene_name": "Synaptotagmin-16",
  "term_id": "UNKNOWN:0003",
  "gene_symbol": "SYT16",
  "gene": "UniProtKB:Q17RD7",
  "term_label": "Unknown cellular component"
}